{
  "gene_name": "Mitochondrial adenyl nucleotide antiporter SLC25A25",
  "term_label": "ATP transport",
  "term_id": "GO:0015867",
  "gene": "UniProtKB:Q6KCM7",
  "gene_symbol": "SLC25A25"
}